{
  "term_label": "plasma membrane",
  "gene_name": "Adenylate cyclase type 5",
  "gene_symbol": "ADCY5",
  "gene": "UniProtKB:O95622",
  "term_id": "GO:0005886"
}